{
  "gene": "UniProtKB:P46019",
  "term_id": "UNKNOWN:0001",
  "gene_name": "Phosphorylase b kinase regulatory subunit alpha, liver isoform",
  "term_label": "Unknown molecular function",
  "gene_symbol": "PHKA2"
}